{
  "gene_symbol": "P2RX5",
  "gene_name": "P2X purinoceptor 5",
  "term_id": "GO:0004931",
  "gene": "UniProtKB:Q93086",
  "term_label": "extracellularly ATP-gated monoatomic cation channel activity"
}